proton-transporting ATP synthase activity, rotational mechanism [GO:0046933] (MF) Sources: RHEA:57722 Definition: Enables the synthesis of ATP from ADP and phosphate by the transfer of protons from one side of a membrane to the other by a rotational mechanism driven by a gradient according to the reaction: ADP + phosphate + 5 H+(out) => ATP + H2O + 4 H+(in). Relationships: is a type of GO:0015252; is a type of ligase activity [GO:0016874]; is part of proton motive force-driven ATP synthesis [GO:0015986] Regulation: positively regulated by positive regulation of proton-transporting ATP synthase activity, rotational mechanism [GO:1905273] Also known as: hydrogen ion transporting ATP synthase activity, rotational mechanism, H+-transporting ATP synthase activity